actin filament branching [GO:0090135] (biological process) Relationships: is_a actin filament organization [GO:0007015] Sources: GOC:ascb_2009, GOC:dph, GOC:tb Definition: The formation of daughter actin filament branches at an angle on the sides of preexisting mother filaments.